{
  "term_id": "UNKNOWN:0003",
  "gene": "UniProtKB:P81277",
  "gene_symbol": "PRLH",
  "term_label": "Unknown cellular component",
  "gene_name": "Prolactin-releasing peptide"
}